nitric-oxide synthase complex [GO:1903958] (cellular component) Also known as: iNOS-S100A8/A9 complex References: PMID:25417112 Sources: GOC:TermGenie, GOC:bhm, GO_REF:0000088 Note: An example of this is NOS2 in human (P35228) in PMID:25417112 (inferred from direct assay). Relationships: is a type of GO:1990204 Subtypes: iNOS-S100A8/A9 complex [GO:1990657] Definition: A protein complex which is capable of nitric-oxide synthase activity.